{
  "gene_name": "FERM and PDZ domain-containing protein 2",
  "gene_symbol": "FRMPD2",
  "term_label": "bicellular tight junction",
  "term_id": "GO:0005923",
  "gene": "UniProtKB:Q68DX3"
}